response to insect [GO:0009625] (biological process) Sources: GOC:hb Relationships: is a type of response to other organism [GO:0051707] Definition: Any process that results in a change in state or activity of a cell or an organism (in terms of movement, secretion, enzyme production, gene expression, etc.) as a result of a stimulus from an insect. Also known as: response to insects